{
  "term_id": "GO:0007283",
  "gene_name": "Tudor domain-containing protein 7",
  "term_label": "spermatogenesis",
  "gene": "UniProtKB:Q8NHU6",
  "gene_symbol": "TDRD7"
}